{
  "term_label": "cell-cell signaling",
  "gene_name": "Gap junction delta-4 protein",
  "gene_symbol": "GJD4",
  "term_id": "GO:0007267",
  "gene": "UniProtKB:Q96KN9"
}